{
  "term_id": "GO:0005874",
  "term_label": "microtubule",
  "gene_name": "Tubulin beta-4B chain",
  "gene_symbol": "TUBB4B",
  "gene": "UniProtKB:P68371"
}